{
  "gene_symbol": "GPR27",
  "term_id": "GO:0004930",
  "gene": "UniProtKB:Q9NS67",
  "gene_name": "Probable G-protein coupled receptor 27",
  "term_label": "G protein-coupled receptor activity"
}